{
  "gene": "UniProtKB:P08910",
  "term_id": "GO:0036126",
  "gene_symbol": "ABHD2",
  "term_label": "sperm flagellum",
  "gene_name": "Monoacylglycerol lipase ABHD2"
}